{
  "gene_symbol": "RSPH10B",
  "gene": "UniProtKB:P0C881",
  "term_label": "Unknown molecular function",
  "term_id": "UNKNOWN:0001",
  "gene_name": "Radial spoke head 10 homolog B"
}